{
  "term_label": "Unknown biological process",
  "gene_symbol": "MFSD4A",
  "gene": "UniProtKB:Q8N468",
  "term_id": "UNKNOWN:0002",
  "gene_name": "Major facilitator superfamily domain-containing protein 4A"
}